{
  "gene_symbol": "FTL",
  "term_label": "cytoplasm",
  "gene": "UniProtKB:P02792",
  "term_id": "GO:0005737",
  "gene_name": "Ferritin light chain"
}